{
  "gene": "UniProtKB:Q04900",
  "gene_symbol": "CD164",
  "gene_name": "Sialomucin core protein 24",
  "term_label": "Unknown molecular function",
  "term_id": "UNKNOWN:0001"
}